{
  "gene_name": "Casein kinase I isoform gamma-3",
  "term_label": "cytoplasm",
  "gene_symbol": "CSNK1G3",
  "gene": "UniProtKB:Q9Y6M4",
  "term_id": "GO:0005737"
}